secalciferol 1-monooxygenase activity [GO:0062185] (MF) Relationships: is a type of monooxygenase activity [GO:0004497] Definition: Catalysis of the reaction:2 H+ + O2 + 2 reduced [adrenodoxin] + secalciferol = calcitetrol + H2O + 2 oxidized [adrenodoxin]. References: PMID:10518789 Sources: RHEA:49064